{
  "gene_name": "Immunoglobulin V-set domain-containing protein (Fragment)",
  "term_id": "GO:0016064",
  "gene_symbol": "A0A0J9YW62",
  "gene": "UniProtKB:A0A0J9YW62",
  "term_label": "immunoglobulin mediated immune response"
}